{
  "gene_symbol": "IFT20",
  "gene_name": "Intraflagellar transport protein 20 homolog",
  "term_id": "UNKNOWN:0001",
  "gene": "UniProtKB:Q8IY31",
  "term_label": "Unknown molecular function"
}